{
  "gene": "UniProtKB:Q8IWB6",
  "term_label": "midbody",
  "term_id": "GO:0030496",
  "gene_symbol": "TEX14",
  "gene_name": "Inactive serine_threonine-protein kinase TEX14"
}